lysosomal enzyme secretion involved in inflammatory response [GO:0002533] (biological process) Relationships: is a type of GO:0033299; BFO_0000050 lysosomal enzyme production involved in inflammatory response [GO:0002393] Definition: The regulated release of lysosomal enzymes by a cell as part of an inflammatory response. Also known as: secretion of lysosomal enzymes involved in acute inflammatory response, secretion of lysosomal enzymes involved in inflammatory response, lysosomal enzyme secretion involved in acute inflammatory response References: PMID:11836514 Sources: GOC:jal